{
  "gene_name": "Immunoglobulin heavy variable 1-69",
  "term_id": "UNKNOWN:0003",
  "term_label": "Unknown cellular component",
  "gene_symbol": "IGHV1-69",
  "gene": "UniProtKB:P01742"
}